{
  "gene_symbol": "IGHV3-38",
  "term_id": "GO:0003823",
  "gene": "UniProtKB:A0A0C4DH36",
  "term_label": "antigen binding",
  "gene_name": "Probable non-functional immunoglobulin heavy variable 3-38"
}